larval serum protein complex [GO:0005616] (cellular component) References: PMID:6781759 Sources: GOC:jl Definition: A multisubunit protein complex which, in Drosophila, is a heterohexamer of three subunits, alpha, beta and gamma. The complex is thought to store amino acids for synthesis of adult proteins. Relationships: is a type of protein-containing complex [GO:0032991]; is part of GO:0005615